{
  "term_label": "defense response to virus",
  "gene": "UniProtKB:Q01629",
  "gene_symbol": "IFITM2",
  "gene_name": "Interferon-induced transmembrane protein 2",
  "term_id": "GO:0051607"
}